{
  "term_id": "GO:0005794",
  "gene_symbol": "TMED4",
  "term_label": "Golgi apparatus",
  "gene_name": "Transmembrane emp24 domain-containing protein 4",
  "gene": "UniProtKB:Q7Z7H5"
}